{
  "gene_name": "Exocyst complex component 3-like protein 2",
  "term_label": "Unknown molecular function",
  "gene": "UniProtKB:Q2M3D2",
  "term_id": "UNKNOWN:0001",
  "gene_symbol": "EXOC3L2"
}